{
  "gene_name": "Putative POM121-like protein 1-like",
  "gene_symbol": "A6NNC1",
  "term_id": "UNKNOWN:0003",
  "term_label": "Unknown cellular component",
  "gene": "UniProtKB:A6NNC1"
}